maintenance of kidney identity [GO:0072005] (biological process) Also known as: maintenance of kidney anlage identity Relationships: is_a maintenance of animal organ identity [GO:0048496]; is part of kidney rudiment formation [GO:0072003] Definition: The process in which the identity of a kidney is maintained. Identity is considered to be the aggregate of characteristics by which a structure is recognized. Sources: GOC:mtg_kidney_jan10